{
  "gene": "UniProtKB:Q9NUG6",
  "term_id": "UNKNOWN:0001",
  "gene_name": "p53 and DNA damage-regulated protein 1",
  "gene_symbol": "PDRG1",
  "term_label": "Unknown molecular function"
}